{
  "term_label": "base-excision repair",
  "gene": "UniProtKB:Q9UIF7",
  "gene_symbol": "MUTYH",
  "term_id": "GO:0006284",
  "gene_name": "Adenine DNA glycosylase"
}